{
  "term_id": "GO:0005886",
  "term_label": "plasma membrane",
  "gene_name": "Free fatty acid receptor 1",
  "gene_symbol": "FFAR1",
  "gene": "UniProtKB:O14842"
}